{
  "gene_symbol": "FILIP1L",
  "term_label": "actin cytoskeleton",
  "gene": "UniProtKB:Q4L180",
  "term_id": "GO:0015629",
  "gene_name": "Filamin A-interacting protein 1-like"
}